{
  "gene_name": "Cysteine-rich hydrophobic domain-containing protein 2",
  "gene": "UniProtKB:Q9UKJ5",
  "term_label": "plasma membrane",
  "term_id": "GO:0005886",
  "gene_symbol": "CHIC2"
}